{
  "gene_symbol": "UVRAG",
  "gene": "UniProtKB:Q9P2Y5",
  "term_label": "endosome",
  "gene_name": "UV radiation resistance-associated gene protein",
  "term_id": "GO:0005768"
}